{
  "gene_symbol": "GNB3",
  "gene_name": "Guanine nucleotide-binding protein G(I)_G(S)_G(T) subunit beta-3",
  "term_label": "heterotrimeric G-protein complex",
  "gene": "UniProtKB:P16520",
  "term_id": "GO:0005834"
}